{
  "gene_symbol": "GRWD1",
  "gene": "UniProtKB:Q9BQ67",
  "term_label": "Unknown molecular function",
  "gene_name": "Glutamate-rich WD repeat-containing protein 1",
  "term_id": "UNKNOWN:0001"
}